{
  "term_id": "GO:0009617",
  "gene_symbol": "TRAV34",
  "gene": "UniProtKB:A0A0B4J273",
  "term_label": "response to bacterium",
  "gene_name": "T cell receptor alpha variable 34"
}